unsaturated chondroitin disaccharide hydrolase activity [GO:0102212] (molecular function) Sources: EC:3.2.1.180, GOC:pz Relationships: is a type of hydrolase activity, hydrolyzing O-glycosyl compounds [GO:0004553] Definition: Catalysis of the reaction: beta-D-4-deoxy-Delta(4)-GlcpA-(1->3)-beta-D-GalpNAc6S + H2O = 5-dehydro-4-deoxy-D-glucuronate + N-acetyl-beta-D-galactosamine 6-sulfate.